sex determination, somatic-gonadal interaction [GO:0007543] (biological process) Also known as: sex determination, somatic/gonadal interaction Definition: The process that mediates the interactions between somatic cells and gonadal cells that ultimately results in the specification of sexual status of the organism. Relationships: is a type of cell communication [GO:0007154]; is part of GO:0007542 Sources: GOC:isa_complete